{
  "gene": "UniProtKB:Q9UPQ4",
  "gene_symbol": "TRIM35",
  "gene_name": "E3 ubiquitin-protein ligase TRIM35",
  "term_id": "GO:0061630",
  "term_label": "ubiquitin protein ligase activity"
}